{
  "term_id": "UNKNOWN:0001",
  "gene_name": "Centromere protein Q",
  "gene_symbol": "CENPQ",
  "term_label": "Unknown molecular function",
  "gene": "UniProtKB:Q7L2Z9"
}